{
  "gene_name": "T cell receptor delta variable 3",
  "term_id": "GO:0019814",
  "gene": "UniProtKB:A0JD37",
  "term_label": "immunoglobulin complex",
  "gene_symbol": "TRDV3"
}